{
  "gene_symbol": "DENND10",
  "gene": "UniProtKB:Q8TCE6",
  "term_id": "GO:0005085",
  "gene_name": "DENN domain-containing protein 10",
  "term_label": "guanyl-nucleotide exchange factor activity"
}